inhibition of dopamine uptake involved in synaptic transmission [GO:0051587] (BP) Sources: GOC:ai Definition: Any process that prevents the activation of the directed movement of dopamine into a cell. Relationships: is a type of negative regulation of dopamine uptake involved in synaptic transmission [GO:0051585]; is_a inhibition of neurotransmitter uptake [GO:0051609] Also known as: inhibition of dopamine import involved in synaptic transmission